D-aspartate transmembrane transporter activity [GO:0140010] (molecular function) References: PMID:7914198 Sources: GO_REF:0000070 Definition: Enables the transfer of D-aspartate from one side of a membrane to the other. Relationships: is a type of dicarboxylic acid transmembrane transporter activity [GO:0005310]; is a type of C4-dicarboxylate transmembrane transporter activity [GO:0015556]; is a type of D-amino acid transmembrane transporter activity [GO:0042943]; is part of D-aspartate transmembrane transport [GO:0070777]